{
  "gene": "UniProtKB:Q6ZVH7",
  "term_label": "cytoplasm",
  "gene_symbol": "ESPNL",
  "gene_name": "Espin-like protein",
  "term_id": "GO:0005737"
}